{
  "gene_symbol": "ETFB",
  "term_id": "GO:0005739",
  "gene": "UniProtKB:P38117",
  "term_label": "mitochondrion",
  "gene_name": "Electron transfer flavoprotein subunit beta"
}